carbon-monoxide oxygenase activity [GO:0008805] (molecular function) Also known as: carbon monoxide oxygenase activity, carbon monoxide oxygenase (cytochrome b-561) activity, carbon monoxide:methylene blue oxidoreductase activity, cytochrome b561, carbon monoxide oxidase activity, carbon monoxide,water:cytochrome b-561 oxidoreductase activity, carbon-monoxide dehydrogenase (cytochrome b-561) Relationships: is a type of GO:0016622 Definition: Catalysis of the reaction: CO + H2O + ferrocytochrome b-561 = CO2 + 2 H+ + 2 ferricytochrome b-561. Sources: GOC:curators, RHEA:48880